{
  "gene_symbol": "HCK",
  "gene": "UniProtKB:P08631",
  "term_label": "non-membrane spanning protein tyrosine kinase activity",
  "gene_name": "Tyrosine-protein kinase HCK",
  "term_id": "GO:0004715"
}